{
  "term_id": "GO:0015175",
  "gene_symbol": "SLC6A19",
  "gene": "UniProtKB:Q695T7",
  "gene_name": "Sodium-dependent neutral amino acid transporter B(0)AT1",
  "term_label": "neutral L-amino acid transmembrane transporter activity"
}